{
  "gene_name": "Calcineurin B homologous protein 3",
  "term_label": "calcium ion binding",
  "gene": "UniProtKB:Q96BS2",
  "gene_symbol": "TESC",
  "term_id": "GO:0005509"
}